{
  "gene": "UniProtKB:Q96CB5",
  "gene_symbol": "C8orf44",
  "term_id": "UNKNOWN:0001",
  "term_label": "Unknown molecular function",
  "gene_name": "Putative uncharacterized protein C8orf44"
}